{
  "gene": "UniProtKB:P39880",
  "term_id": "GO:0006357",
  "gene_name": "Homeobox protein cut-like 1",
  "term_label": "regulation of transcription by RNA polymerase II",
  "gene_symbol": "CUX1"
}